negative regulation of meiotic cell cycle process involved in oocyte maturation [GO:1904145] (biological process) Definition: Any process that stops, prevents or reduces the frequency, rate or extent of meiotic cell cycle process involved in oocyte maturation. References: PMID:22674394 Sources: GOC:TermGenie, GO_REF:0000058 Also known as: down regulation of meiotic cell cycle process involved in oocyte maturation, down-regulation of meiotic cell cycle process involved in oocyte maturation, downregulation of meiotic cell cycle process involved in oocyte maturation, inhibition of meiotic cell cycle process involved in oocyte maturation Relationships: is a type of negative regulation of cell cycle process [GO:0010948]; is a type of GO:0051447; is_a negative regulation of oocyte maturation [GO:1900194]; is_a regulation of meiotic cell cycle process involved in oocyte maturation [GO:1903538]; negatively regulates meiotic cell cycle process involved in oocyte maturation [GO:1903537]